{
  "term_id": "UNKNOWN:0001",
  "gene_name": "GREB1-like protein",
  "term_label": "Unknown molecular function",
  "gene": "UniProtKB:Q9C091",
  "gene_symbol": "GREB1L"
}